{
  "term_id": "UNKNOWN:0001",
  "gene_name": "Protein NDRG3",
  "term_label": "Unknown molecular function",
  "gene_symbol": "NDRG3",
  "gene": "UniProtKB:Q9UGV2"
}